tRNA methylthiolation [GO:0035600] (biological process) Relationships: is a type of tRNA modification [GO:0006400] Definition: The addition of a methylthioether group (-SCH3) to a nucleotide in a tRNA molecule. References: PMID:20472640